{
  "term_id": "GO:0007288",
  "gene_name": "Tubulin polyglutamylase TTLL5",
  "gene": "UniProtKB:Q6EMB2",
  "term_label": "sperm axoneme assembly",
  "gene_symbol": "TTLL5"
}